{
  "term_id": "UNKNOWN:0002",
  "gene_symbol": "FAM200A",
  "term_label": "Unknown biological process",
  "gene": "UniProtKB:Q8TCP9",
  "gene_name": "Protein FAM200A"
}